{
  "gene": "UniProtKB:A6NC62",
  "gene_name": "Putative RBAK downstream neighbor protein",
  "term_id": "UNKNOWN:0003",
  "gene_symbol": "RBAKDN",
  "term_label": "Unknown cellular component"
}